{
  "term_id": "UNKNOWN:0002",
  "gene": "UniProtKB:Q8N8V8",
  "gene_symbol": "TMEM105",
  "term_label": "Unknown biological process",
  "gene_name": "Transmembrane protein 105"
}